macrophage antigen processing and presentation [GO:0002472] (biological process) Regulation: regulated by regulation of macrophage antigen processing and presentation [GO:0002616]; negatively regulated by GO:0002617; positively regulated by positive regulation of macrophage antigen processing and presentation [GO:0002618] Relationships: is a type of antigen processing and presentation [GO:0019882] References: PMID:15771591 Sources: GOC:add, ISBN:0781735149 Definition: The process in which a macrophage expresses antigen (peptide or lipid) on its cell surface in association with an MHC protein complex.